{
  "term_label": "regulation of RNA splicing",
  "term_id": "GO:0043484",
  "gene_symbol": "CLK3",
  "gene": "UniProtKB:P49761",
  "gene_name": "Dual specificity protein kinase CLK3"
}